protein-N(PI)-phosphohistidine-sorbose phosphotransferase system transporter activity [GO:0022871] (molecular function) Relationships: is a type of protein-N(PI)-phosphohistidine-sugar phosphotransferase activity [GO:0008982]; is a type of D-glucose transmembrane transporter activity [GO:0055056] Also known as: sorbose PTS transporter activity Definition: Catalysis of the PEP-dependent, phosphoryl transfer-driven transport of substances across a membrane. The transport happens by catalysis of the reaction: protein N-phosphohistidine + sorbose(out) = protein histidine + sorbose phosphate(in). This differs from primary and secondary active transport in that the solute is modified during transport. References: PMID:10613875 Sources: GOC:mtg_transport, RHEA:49296